{
  "gene": "UniProtKB:P46940",
  "term_id": "GO:0010761",
  "gene_name": "Ras GTPase-activating-like protein IQGAP1",
  "term_label": "fibroblast migration",
  "gene_symbol": "IQGAP1"
}